{
  "gene_name": "Protocadherin gamma-B4",
  "term_label": "cell adhesion molecule binding",
  "gene": "UniProtKB:Q9UN71",
  "term_id": "GO:0050839",
  "gene_symbol": "PCDHGB4"
}